{
  "gene_name": "Uncharacterized protein C3orf85",
  "gene_symbol": "C3orf85",
  "term_id": "UNKNOWN:0001",
  "term_label": "Unknown molecular function",
  "gene": "UniProtKB:A0A1B0GTC6"
}